protein histidine phosphatase activity [GO:0101006] (molecular function) Relationships: is a type of phosphoprotein phosphatase activity [GO:0004721]; is a type of hydrolase activity, acting on acid phosphorus-nitrogen bonds [GO:0016825] Definition: Catalysis of the reaction: protein histidine phosphate + H2O = protein histidine + phosphate. Note: This eukaryotic enzyme dephosphorylates phosphorylated histidine residues within proteins and peptides. The enzyme acts on phosphate groups attached to both the pros- (RHEA:47964) and tele- (RHEA:47960) nitrogen atoms, but the pros- position is somewhat preferred (by a factor of two at the most) (EC:3.9.1.3). Sources: EC:3.9.1.3 Also known as: phosphohistidine phosphatase activity